tetrahydrobiopterin biosynthetic process [GO:0006729] (biological process) Also known as: 5,6,7,8-tetrahydrobiopterin biosynthetic process, tetrahydrobiopterin anabolism, tetrahydrobiopterin biosynthesis, tetrahydrobiopterin formation, tetrahydrobiopterin synthesis Sources: ISBN:0198506732 Relationships: is a type of diol biosynthetic process [GO:0034312]; is_a pteridine-containing compound biosynthetic process [GO:0042559]; is a type of GO:0046146 Definition: The chemical reactions and pathways resulting in the formation of tetrahydrobiopterin, the reduced form of biopterin (2-amino-4-hydroxy-6-(1,2-dihydroxypropyl)-pteridine). It functions as a hydroxylation coenzyme, e.g. in the conversion of phenylalanine to tyrosine.